{
  "term_label": "cell surface receptor signaling pathway",
  "term_id": "GO:0007166",
  "gene_name": "Membrane-spanning 4-domains subfamily A member 13",
  "gene": "UniProtKB:Q5J8X5",
  "gene_symbol": "MS4A13"
}